thymic stromal lymphopoietin production [GO:0071925] (biological process) Definition: The appearance of thymic stromal lymphopoietin (TSLP) due to biosynthesis or secretion following a cellular stimulus, resulting in an increase in its intracellular or extracellular levels. References: PMID:17129180 Sources: GOC:mah Relationships: is a type of chemokine production [GO:0032602] Also known as: TSLP production